{
  "gene_name": "Cystatin-8",
  "term_label": "Unknown biological process",
  "gene_symbol": "CST8",
  "term_id": "UNKNOWN:0002",
  "gene": "UniProtKB:O60676"
}